{
  "gene": "UniProtKB:P22492",
  "gene_symbol": "H1-6",
  "gene_name": "Histone H1t",
  "term_id": "GO:0005634",
  "term_label": "nucleus"
}